{
  "term_id": "GO:0035556",
  "gene_name": "Serine_threonine-protein kinase 32B",
  "gene_symbol": "STK32B",
  "gene": "UniProtKB:Q9NY57",
  "term_label": "intracellular signal transduction"
}